{
  "term_label": "RNA polymerase II cis-regulatory region sequence-specific DNA binding",
  "gene": "UniProtKB:P09067",
  "gene_name": "Homeobox protein Hox-B5",
  "term_id": "GO:0000978",
  "gene_symbol": "HOXB5"
}